{
  "term_label": "regulation of gene expression",
  "term_id": "GO:0010468",
  "gene_name": "Developmental pluripotency-associated 5 protein",
  "gene_symbol": "DPPA5",
  "gene": "UniProtKB:A6NC42"
}